{
  "term_label": "cell differentiation",
  "gene_name": "Follistatin-related protein 4",
  "gene_symbol": "FSTL4",
  "gene": "UniProtKB:Q6MZW2",
  "term_id": "GO:0030154"
}